{
  "gene": "UniProtKB:P06865",
  "gene_symbol": "HEXA",
  "term_label": "ganglioside catabolic process",
  "term_id": "GO:0006689",
  "gene_name": "Beta-hexosaminidase subunit alpha"
}